{
  "term_id": "GO:0006099",
  "term_label": "tricarboxylic acid cycle",
  "gene_symbol": "MDH1",
  "gene": "UniProtKB:P40925",
  "gene_name": "Malate dehydrogenase, cytoplasmic"
}